{
  "gene_name": "Phosphatase and actin regulator 1",
  "gene": "UniProtKB:Q9C0D0",
  "gene_symbol": "PHACTR1",
  "term_label": "stress fiber assembly",
  "term_id": "GO:0043149"
}